{
  "term_id": "GO:0006670",
  "gene_name": "Sphingosine-1-phosphate phosphatase 2",
  "term_label": "sphingosine metabolic process",
  "gene": "UniProtKB:Q8IWX5",
  "gene_symbol": "SGPP2"
}